sulfolactate sulfo-lyase activity [GO:0034010] (molecular function) Sources: EC:4.4.1.24, RHEA:21428 Definition: Catalysis of the reaction: 3-sulfolactate = pyruvate + sulfite. Relationships: is_a carbon-sulfur lyase activity [GO:0016846] Also known as: 3-sulfolactate bisulfite-lyase (pyruvate-forming) activity, 3-sulfolactate bisulfite-lyase activity, Suy, SuyAB